{
  "gene_name": "Endosialin",
  "gene": "UniProtKB:Q9HCU0",
  "term_label": "external side of plasma membrane",
  "term_id": "GO:0009897",
  "gene_symbol": "CD248"
}